rostrocaudal neural tube patterning [GO:0021903] (biological process) References: PMID:11262869 Sources: GOC:cls, GOC:dgh, GOC:dph, GOC:jid, GO_REF:0000021 Also known as: anterior-posterior neural tube patterning Relationships: is a type of anterior/posterior pattern specification [GO:0009952]; is part of GO:0021532 Definition: The process in which the neural tube is divided into specific regions along the rostrocaudal axis.